{
  "gene_symbol": "GGNBP2",
  "gene": "UniProtKB:Q9H3C7",
  "term_id": "GO:0005634",
  "gene_name": "Gametogenetin-binding protein 2",
  "term_label": "nucleus"
}